{
  "gene_name": "Cyclin-dependent kinase inhibitor 2A",
  "term_id": "GO:0005634",
  "term_label": "nucleus",
  "gene": "UniProtKB:P42771",
  "gene_symbol": "CDKN2A"
}